{
  "term_label": "centrosome",
  "term_id": "GO:0005813",
  "gene_name": "Centrin-1",
  "gene": "UniProtKB:Q12798",
  "gene_symbol": "CETN1"
}